{
  "term_label": "regulation of apoptotic process",
  "gene_name": "Protein BEX2",
  "term_id": "GO:0042981",
  "gene": "UniProtKB:Q9BXY8",
  "gene_symbol": "BEX2"
}